{
  "term_label": "transcription initiation at RNA polymerase I promoter",
  "gene_name": "Putative RRN3-like protein RRN3P2",
  "term_id": "GO:0006361",
  "gene": "UniProtKB:A6NIE6",
  "gene_symbol": "RRN3P2"
}